{
  "gene": "UniProtKB:Q5HYC2",
  "term_id": "UNKNOWN:0002",
  "gene_symbol": "KIAA2026",
  "term_label": "Unknown biological process",
  "gene_name": "Uncharacterized protein KIAA2026"
}